embryonic viscerocranium morphogenesis [GO:0048703] (biological process) Also known as: embryonic pharyngeal skeleton morphogenesis References: PMID:16049113 Sources: GOC:dsf, GOC:jid Relationships: is a type of embryonic morphogenesis [GO:0048598]; is part of GO:0048701 Definition: The process in which the anatomical structures of the viscerocranium are generated and organized during the embryonic phase. The viscerocranium is the part of the skull comprising the facial bones.